{
  "gene": "UniProtKB:Q107X0",
  "gene_name": "Putative protein KRIP1",
  "term_id": "UNKNOWN:0002",
  "term_label": "Unknown biological process",
  "gene_symbol": "KLKP1"
}